{
  "gene_symbol": "RAP1GDS1",
  "term_label": "cytosol",
  "gene_name": "Rap1 GTPase-GDP dissociation stimulator 1",
  "term_id": "GO:0005829",
  "gene": "UniProtKB:P52306"
}